{
  "term_id": "GO:0006888",
  "gene": "UniProtKB:P53611",
  "gene_symbol": "RABGGTB",
  "gene_name": "Geranylgeranyl transferase type-2 subunit beta",
  "term_label": "endoplasmic reticulum to Golgi vesicle-mediated transport"
}